regulation of protein localization to mitotic spindle pole body [GO:1902542] (biological process) Subtypes: GO:1902543 Definition: Any process that modulates the frequency, rate or extent of protein localization to mitotic spindle pole body. Relationships: is a type of regulation of protein localization to spindle pole body [GO:1902363]; regulates protein localization to mitotic spindle pole body [GO:1902440] Also known as: regulation of protein localisation to mitotic spindle pole body References: PMID:22809626 Sources: GOC:TermGenie